{
  "gene_name": "Olfactory receptor 5AK2",
  "gene_symbol": "OR5AK2",
  "gene": "UniProtKB:Q8NH90",
  "term_label": "sensory perception of smell",
  "term_id": "GO:0007608"
}